{
  "term_id": "GO:0016264",
  "term_label": "gap junction assembly",
  "gene": "UniProtKB:P29033",
  "gene_symbol": "GJB2",
  "gene_name": "Gap junction beta-2 protein"
}